{
  "gene": "UniProtKB:Q8NH02",
  "gene_symbol": "OR2T29",
  "term_id": "GO:0050911",
  "gene_name": "Olfactory receptor 2T29",
  "term_label": "detection of chemical stimulus involved in sensory perception of smell"
}